{
  "gene_name": "SPARC-like protein 1",
  "term_label": "extracellular matrix",
  "gene": "UniProtKB:Q14515",
  "gene_symbol": "SPARCL1",
  "term_id": "GO:0031012"
}